positive regulation of endothelial microparticle formation [GO:2000337] (biological process) Also known as: positive regulation of endothelial microparticle generation, positive regulation of endothelial microparticle release Sources: GOC:BHF, GOC:mah Definition: Any process that activates or increases the frequency, rate or extent of endothelial microparticle formation. Relationships: is a type of positive regulation of blood microparticle formation [GO:2000334]; is a type of regulation of endothelial microparticle formation [GO:2000335]; positively regulates GO:0072565